{
  "term_id": "GO:0034657",
  "gene_name": "Ran-binding protein 10",
  "gene": "UniProtKB:Q6VN20",
  "term_label": "GID complex",
  "gene_symbol": "RANBP10"
}